thiamine diphosphate biosynthetic process [GO:0009229] (biological process) Definition: The chemical reactions and pathways resulting in the formation of thiamine diphosphate, a derivative of thiamine (vitamin B1) which acts as a coenzyme in a range of processes including the Krebs cycle. Regulation: regulated by regulation of thiamine diphosphate biosynthetic process [GO:0070616]; negatively regulated by negative regulation of thiamine diphosphate biosynthetic process [GO:0070617] Sources: GOC:jl, ISBN:0140512713 Also known as: TPP biosynthesis, TPP biosynthetic process, thiamin diphosphate biosynthetic process, thiamin pyrophosphate biosynthesis, thiamin pyrophosphate biosynthetic process, thiamine diphosphate anabolism, thiamine diphosphate biosynthesis, thiamine diphosphate formation, thiamine diphosphate synthesis, thiamine pyrophosphate biosynthesis, thiamine pyrophosphate biosynthetic process Relationships: is a type of GO:0042357; is a type of GO:0042724; is a type of GO:0090407